{
  "gene_symbol": "NPY2R",
  "gene": "UniProtKB:P49146",
  "term_id": "GO:0005886",
  "gene_name": "Neuropeptide Y receptor type 2",
  "term_label": "plasma membrane"
}